lithium ion transmembrane transport [GO:0090452] (BP) Sources: GOC:tb Also known as: lithium ion uptake, lithium ion import Subtypes: GO:0010352 Relationships: is a type of lithium ion transport [GO:0010351]; is_a monoatomic cation transmembrane transport [GO:0098655] Definition: The directed movement of lithium ions (Li+) across a membrane.